{
  "gene": "UniProtKB:Q9HB65",
  "term_id": "GO:0042795",
  "gene_name": "RNA polymerase II elongation factor ELL3",
  "term_label": "snRNA transcription by RNA polymerase II",
  "gene_symbol": "ELL3"
}